{
  "term_label": "Unknown molecular function",
  "gene": "UniProtKB:P60827",
  "gene_symbol": "C1QTNF8",
  "term_id": "UNKNOWN:0001",
  "gene_name": "Complement C1q tumor necrosis factor-related protein 8"
}